{
  "gene_name": "Probable non-functional T cell receptor beta variable 23-1",
  "gene": "UniProtKB:A0A0A0MS06",
  "gene_symbol": "TRBV23-1",
  "term_label": "cell surface receptor signaling pathway",
  "term_id": "GO:0007166"
}